{
  "term_label": "epigenetic regulation of gene expression",
  "gene_name": "Zinc finger protein 335",
  "gene": "UniProtKB:Q9H4Z2",
  "gene_symbol": "ZNF335",
  "term_id": "GO:0040029"
}